positive regulation of complement activation [GO:0045917] (biological process) Definition: Any process that activates or increases the frequency, rate or extent of complement activation. Also known as: positive regulation of complement cascade, up regulation of complement activation, up-regulation of complement activation, upregulation of complement activation, activation of complement activation, stimulation of complement activation Subtypes: positive regulation of complement activation, lectin pathway [GO:0001870], positive regulation of activation of membrane attack complex [GO:0001970], GO:0045958, GO:0045960 Sources: GOC:go_curators Relationships: is a type of positive regulation of immune effector process [GO:0002699]; is a type of positive regulation of humoral immune response [GO:0002922]; is a type of regulation of complement activation [GO:0030449]; positively regulates GO:0006956